{
  "gene_symbol": "HOXA7",
  "term_id": "GO:0009952",
  "term_label": "anterior/posterior pattern specification",
  "gene": "UniProtKB:P31268",
  "gene_name": "Homeobox protein Hox-A7"
}